{
  "gene_name": "Protein FAM118A",
  "gene": "UniProtKB:Q9NWS6",
  "term_label": "Unknown biological process",
  "gene_symbol": "FAM118A",
  "term_id": "UNKNOWN:0002"
}